{
  "gene_name": "Putative uncharacterized protein NTM-AS1",
  "term_id": "UNKNOWN:0003",
  "gene_symbol": "NTM-AS1",
  "gene": "UniProtKB:Q6ZSK4",
  "term_label": "Unknown cellular component"
}